positive regulation of tolerance induction to tumor cell [GO:0002845] (biological process) Definition: Any process that activates or increases the frequency, rate, or extent of tolerance induction to tumor cell. Sources: GOC:add Also known as: positive regulation of tolerance induction to tumour cell, up regulation of tolerance induction to tumor cell, up-regulation of tolerance induction to tumor cell, upregulation of tolerance induction to tumor cell, activation of tolerance induction to tumor cell, stimulation of tolerance induction to tumor cell Relationships: is_a GO:0002660; is a type of positive regulation of immune response to tumor cell [GO:0002839]; is a type of regulation of tolerance induction to tumor cell [GO:0002843]; positively regulates GO:0002413 Subtypes: positive regulation of T cell tolerance induction to tumor cell [GO:0002848]